ocellus photoreceptor cell development [GO:0042463] (biological process) References: PMID:11542766 Sources: GOC:jl, ISBN:0192800981 Definition: Development of photoreceptors, sensory cells that react to the presence of light, found in the ocellus. Also known as: non-eye photoreceptor development Relationships: is a type of photoreceptor cell development [GO:0042461]; is part of GO:0042705